{
  "term_id": "GO:0000978",
  "gene": "UniProtKB:O60315",
  "gene_symbol": "ZEB2",
  "term_label": "RNA polymerase II cis-regulatory region sequence-specific DNA binding",
  "gene_name": "Zinc finger E-box-binding homeobox 2"
}